{
  "gene_symbol": "SP140L",
  "term_label": "nucleus",
  "term_id": "GO:0005634",
  "gene_name": "Nuclear body protein SP140-like protein",
  "gene": "UniProtKB:Q9H930"
}